{
  "term_label": "positive regulation of type I interferon production",
  "gene_symbol": "TBK1",
  "gene_name": "Serine_threonine-protein kinase TBK1",
  "gene": "UniProtKB:Q9UHD2",
  "term_id": "GO:0032481"
}